{
  "term_label": "plasma membrane",
  "term_id": "GO:0005886",
  "gene_symbol": "SLC5A9",
  "gene_name": "Sodium_glucose cotransporter 4",
  "gene": "UniProtKB:Q2M3M2"
}